myosin III complex [GO:0042385] (cellular component) Relationships: is a type of unconventional myosin complex [GO:0016461] Definition: A myosin complex containing a class III myosin heavy chain and associated light chains; myosin III is monomeric myosin that serves as a link between the cytoskeleton and the signaling complex involved in phototransduction, and differs from all other myosins in having an N-terminal kinase domain. References: PMID:33718386 Sources: GOC:jl